regulation of amine metabolic process [GO:0033238] (biological process) Definition: Any process that modulates the frequency, rate or extent of the chemical reactions and pathways by which individual cells transform amines. Sources: GOC:mah Also known as: regulation of amine metabolism, regulation of cellular amine metabolic process Relationships: is a type of regulation of metabolic process [GO:0019222]; regulates amine metabolic process [GO:0009308] Subtypes: regulation of polyamine biosynthetic process [GO:0010967], GO:0033239, positive regulation of amine metabolic process [GO:0033240], regulation of amine catabolic process [GO:0033241], GO:0042069, regulation of acetylcholine metabolic process [GO:0060408], regulation of methane biosynthetic process from dimethylamine [GO:1900318], regulation of methane biosynthetic process from trimethylamine [GO:1900330], regulation of methane biosynthetic process from methylamine [GO:1900348]